{
  "term_label": "Unknown biological process",
  "gene": "UniProtKB:Q9UHL3",
  "term_id": "UNKNOWN:0002",
  "gene_symbol": "FAM153A",
  "gene_name": "Protein FAM153A"
}